{
  "gene_symbol": "RCN3",
  "term_label": "endoplasmic reticulum",
  "gene_name": "Reticulocalbin-3",
  "term_id": "GO:0005783",
  "gene": "UniProtKB:Q96D15"
}